{
  "gene_symbol": "DCAF6",
  "gene_name": "DDB1- and CUL4-associated factor 6",
  "term_label": "cytoplasm",
  "term_id": "GO:0005737",
  "gene": "UniProtKB:Q58WW2"
}